{
  "term_label": "cell periphery",
  "term_id": "GO:0071944",
  "gene": "UniProtKB:Q6UX34",
  "gene_symbol": "SNORC",
  "gene_name": "Protein SNORC"
}